{
  "gene_name": "Orphan sodium- and chloride-dependent neurotransmitter transporter NTT5",
  "gene": "UniProtKB:Q9GZN6",
  "gene_symbol": "SLC6A16",
  "term_label": "Unknown molecular function",
  "term_id": "UNKNOWN:0001"
}